oligosaccharide transport [GO:0015772] (biological process) Relationships: is a type of GO:0008643 Definition: The directed movement of oligosaccharides into, out of or within a cell, or between cells, by means of some agent such as a transporter or pore. Oligosaccharides are molecules with between two and (about) 20 monosaccharide residues connected by glycosidic linkages. Subtypes: disaccharide transport [GO:0015766], GO:0033156, GO:2001088, GO:2001098, pentasaccharide transport [GO:2001100], hexasaccharide transport [GO:2001102], heptasaccharide transport [GO:2001104] Sources: GOC:ai